{
  "term_id": "GO:0042274",
  "gene": "UniProtKB:P62081",
  "gene_symbol": "RPS7",
  "gene_name": "Small ribosomal subunit protein eS7",
  "term_label": "ribosomal small subunit biogenesis"
}